{
  "gene_name": "4-trimethylaminobutyraldehyde dehydrogenase",
  "term_label": "Unknown cellular component",
  "term_id": "UNKNOWN:0003",
  "gene": "UniProtKB:P49189",
  "gene_symbol": "ALDH9A1"
}